{
  "gene_symbol": "ANGEL1",
  "gene": "UniProtKB:Q9UNK9",
  "gene_name": "Protein angel homolog 1",
  "term_label": "Unknown cellular component",
  "term_id": "UNKNOWN:0003"
}